{
  "term_label": "transcription factor TFIID complex",
  "gene": "UniProtKB:P49848",
  "gene_name": "Transcription initiation factor TFIID subunit 6",
  "gene_symbol": "TAF6",
  "term_id": "GO:0005669"
}